{
  "gene_symbol": "PCDHB12",
  "gene": "UniProtKB:Q9Y5F1",
  "term_label": "cell adhesion molecule binding",
  "gene_name": "Protocadherin beta-12",
  "term_id": "GO:0050839"
}